{
  "gene_symbol": "SIRT4",
  "gene_name": "NAD-dependent protein lipoamidase sirtuin-4, mitochondrial",
  "gene": "UniProtKB:Q9Y6E7",
  "term_id": "GO:0005759",
  "term_label": "mitochondrial matrix"
}